{
  "gene_name": "Putative cytosolic acyl coenzyme A thioester hydrolase-like",
  "term_id": "GO:0052816",
  "gene_symbol": "ACOT7L",
  "term_label": "long-chain fatty acyl-CoA hydrolase activity",
  "gene": "UniProtKB:Q6ZUV0"
}